{
  "gene_name": "UDP-glucuronosyltransferase 1-6",
  "gene": "UniProtKB:P19224",
  "term_id": "GO:0004857",
  "term_label": "enzyme inhibitor activity",
  "gene_symbol": "UGT1A6"
}